ATP:ADP antiporter activity [GO:0005471] (molecular function) Definition: Catalysis of the reaction: ATP(out) + ADP(in) = ATP(in) + ADP(out). Sources: TC:2.A.29.1.1 Also known as: ADP/ATP carrier protein, ADP/ATP translocase, ATP/ADP exchange, ATP/ADP exchanger, adenine nucleotide translocase Relationships: is a type of ATP transmembrane transporter activity [GO:0005347]; is a type of GO:0015217; is_a antiporter activity [GO:0015297]